{
  "gene_symbol": "FRG1",
  "gene": "UniProtKB:Q14331",
  "gene_name": "Protein FRG1",
  "term_id": "UNKNOWN:0002",
  "term_label": "Unknown biological process"
}